{
  "gene_name": "NAD-dependent protein deacylase sirtuin-5, mitochondrial",
  "term_id": "GO:0005634",
  "gene_symbol": "SIRT5",
  "gene": "UniProtKB:Q9NXA8",
  "term_label": "nucleus"
}